{
  "term_label": "Unknown molecular function",
  "gene_name": "Putative tenascin-XA",
  "gene": "UniProtKB:Q16473",
  "term_id": "UNKNOWN:0001",
  "gene_symbol": "TNXA"
}